semicircular canal formation [GO:0060876] (biological process) Relationships: is a type of tube formation [GO:0035148]; is part of GO:0048752 Sources: GOC:dph, GOC:sdb_2009, GOC:tb Definition: The developmental process pertaining to the initial formation of the semicircular canal from the otic vesicle. This process begins with the regionalization of the vesicle that specifies the area where the vesicles will form and continues through the process of fusion which forms the initial tubes.